{
  "gene": "UniProtKB:P20941",
  "term_label": "photoreceptor outer segment",
  "gene_name": "Phosducin",
  "gene_symbol": "PDC",
  "term_id": "GO:0001750"
}